signaling adaptor activity [GO:0035591] (molecular function) Subtypes: GO:0005078, JAK pathway signal transduction adaptor activity [GO:0008269], GO:0030159 Note: A signaling adaptor can bring together both protein and non-protein molecules within a signaling pathway. Scaffold proteins act in at least four ways: tethering signaling components, localizing these components to specific areas of the cell, regulating signal transduction by coordinating positive and negative feedback signals, and insulating correct signaling proteins from competing proteins (PMID:19104498). References: PMID:19104498 Sources: GOC:bf Relationships: is a type of GO:0030674 Also known as: signaling protein recruiting activity, signalling adaptor activity, signaling scaffold activity Definition: The binding activity of a molecule that brings together two or more molecules in a signaling pathway, permitting those molecules to function in a coordinated way. Adaptor molecules themselves do not have catalytic activity.